nitrogen-oxygen lyase activity [GO:0141122] (MF) Sources: EC:4.8.1.- Subtypes: phenylacetaldoxime dehydratase activity [GO:0018814], aliphatic aldoxime dehydratase activity [GO:0034013], indoleacetaldoxime dehydratase activity [GO:0047720] Relationships: is a type of lyase activity [GO:0016829] Definition: Catalysis of the breakage of a nitrogen-oxygen bond by means other than hydrolysis and oxidation.